glucomannan catabolic process [GO:2000884] (biological process) Regulation: regulated by GO:2000898; RO_0002212 by negative regulation of glucomannan catabolic process [GO:2000907]; positively regulated by positive regulation of glucomannan catabolic process [GO:2000908] Relationships: is a type of polysaccharide catabolic process [GO:0000272]; is a type of glucomannan metabolic process [GO:0010391] Definition: The chemical reactions and pathways resulting in the breakdown of a glucomannan. Sources: GOC:mengo_curators Also known as: glucomannan catabolism